{
  "gene_symbol": "NPIPA7",
  "term_id": "UNKNOWN:0002",
  "term_label": "Unknown biological process",
  "gene_name": "Nuclear pore complex-interacting protein family member A7",
  "gene": "UniProtKB:E9PJI5"
}